{
  "term_label": "plasma membrane",
  "gene_symbol": "TRPM4",
  "gene_name": "Transient receptor potential cation channel subfamily M member 4",
  "gene": "UniProtKB:Q8TD43",
  "term_id": "GO:0005886"
}